{
  "term_label": "Golgi apparatus",
  "gene": "UniProtKB:Q15363",
  "gene_name": "Transmembrane emp24 domain-containing protein 2",
  "gene_symbol": "TMED2",
  "term_id": "GO:0005794"
}